regulation of isotype switching to IgG isotypes [GO:0048302] (biological process) Sources: GOC:jid Also known as: regulation of class switch recombination to IgG isotypes, regulation of class switching to IgG isotypes, regulation of isotype switch recombination to IgG isotypes Relationships: is a type of regulation of isotype switching [GO:0045191]; regulates isotype switching to IgG isotypes [GO:0048291] Definition: Any process that modulates the frequency, rate or extent of isotype switching to IgG isotypes. Subtypes: GO:0048303, positive regulation of isotype switching to IgG isotypes [GO:0048304]